{
  "term_id": "GO:0000812",
  "term_label": "Swr1 complex",
  "gene_symbol": "RUVBL1",
  "gene_name": "RuvB-like 1",
  "gene": "UniProtKB:Q9Y265"
}